{
  "term_label": "Unknown molecular function",
  "gene": "UniProtKB:A0A0A0MT78",
  "gene_name": "T cell receptor beta joining 2-7",
  "term_id": "UNKNOWN:0001",
  "gene_symbol": "TRBJ2-7"
}